{
  "term_id": "GO:0060271",
  "gene_name": "Centromere protein J",
  "gene": "UniProtKB:Q9HC77",
  "gene_symbol": "CENPJ",
  "term_label": "cilium assembly"
}